{
  "gene": "UniProtKB:Q13478",
  "term_label": "cell surface",
  "term_id": "GO:0009986",
  "gene_name": "Interleukin-18 receptor 1",
  "gene_symbol": "IL18R1"
}